{
  "term_label": "transcription initiation at mitochondrial promoter",
  "gene_symbol": "TFB1M",
  "term_id": "GO:0006391",
  "gene_name": "Dimethyladenosine transferase 1, mitochondrial",
  "gene": "UniProtKB:Q8WVM0"
}